lysyl-tRNA aminoacylation [GO:0006430] (biological process) Relationships: is a type of tRNA aminoacylation for protein translation [GO:0006418] Definition: The process of coupling lysine to lysyl-tRNA, catalyzed by lysyl-tRNA synthetase. The lysyl-tRNA synthetase is a class-II synthetase. The activated amino acid is transferred to the 3'-OH group of a lysine-accetping tRNA. Subtypes: mitochondrial lysyl-tRNA aminoacylation [GO:0070154] Sources: GOC:mcc, ISBN:0716730510